{
  "gene": "UniProtKB:Q5BJH7",
  "term_id": "GO:0006888",
  "gene_name": "Protein YIF1B",
  "term_label": "endoplasmic reticulum to Golgi vesicle-mediated transport",
  "gene_symbol": "YIF1B"
}